{
  "gene_name": "Putative uncharacterized protein ARHGAP5-AS1",
  "term_label": "Unknown molecular function",
  "gene_symbol": "ARHGAP5-AS1",
  "gene": "UniProtKB:Q96IT6",
  "term_id": "UNKNOWN:0001"
}